{
  "term_id": "GO:0017128",
  "gene_symbol": "ANO7",
  "term_label": "phospholipid scramblase activity",
  "gene": "UniProtKB:Q6IWH7",
  "gene_name": "Anoctamin-7"
}